{
  "term_label": "Unknown molecular function",
  "gene_name": "T cell receptor gamma joining P2 (Fragment)",
  "gene_symbol": "TRGJP2",
  "gene": "UniProtKB:A0A0A0MT84",
  "term_id": "UNKNOWN:0001"
}